{
  "gene": "UniProtKB:Q6ZMY3",
  "term_id": "GO:0141196",
  "gene_symbol": "SPOCD1",
  "term_label": "transposable element silencing by piRNA-mediated DNA methylation",
  "gene_name": "SPOC domain-containing protein 1"
}